{
  "term_id": "UNKNOWN:0003",
  "term_label": "Unknown cellular component",
  "gene_symbol": "TRAC",
  "gene": "UniProtKB:P01848",
  "gene_name": "T cell receptor alpha chain constant"
}